3-oxolaurate decarboxylase activity [GO:0050410] (molecular function) Also known as: 3-oxododecanoate carboxy-lyase (2-undecanone-forming), 3-oxododecanoate carboxy-lyase activity, beta-ketoacyl decarboxylase activity, beta-ketolaurate decarboxylase activity Sources: EC:4.1.1.56, RHEA:13385 Definition: Catalysis of the reaction: 3-oxododecanoate + H+ = 2-undecanone + CO2. Also decarboxylates other C14 to C16 oxo acids. Relationships: is a type of carboxy-lyase activity [GO:0016831]